cis-1,2-dihydrobenzene-1,2-diol dehydrogenase activity [GO:0018504] (MF) Definition: Catalysis of the reaction: cis-1,2-dihydrobenzene-1,2-diol + NAD+ = catechol + NADH + H+. Sources: EC:1.3.1.19 Also known as: cis-1,2-dihydrobenzene-1,2-diol:NAD+ oxidoreductase activity, cis-1,2-dihydrocyclohexa-3,5-diene (nicotinamide adenine dinucleotide) oxidoreductase activity, cis-benzene glycol dehydrogenase activity Relationships: is a type of oxidoreductase activity, acting on the CH-CH group of donors, NAD or NADP as acceptor [GO:0016628]